{
  "gene_name": "Corticotropin-releasing factor receptor 1",
  "term_id": "GO:0005886",
  "gene": "UniProtKB:P34998",
  "term_label": "plasma membrane",
  "gene_symbol": "CRHR1"
}